{
  "gene_name": "F-box only protein 16",
  "term_label": "Unknown cellular component",
  "term_id": "UNKNOWN:0003",
  "gene_symbol": "FBXO16",
  "gene": "UniProtKB:Q8IX29"
}